alkanesulfonate metabolic process [GO:0019694] (biological process) Sources: GOC:ai Definition: The chemical reactions and pathways involving alkanesulfonates, the anion of alkanesulfonic acids, sulfonic acid derivatives containing an aliphatic hydrocarbon group. Relationships: is a type of organic acid metabolic process [GO:0006082]; is_a GO:0006790 Also known as: alkanesulfonate metabolism, alkanesulphonate metabolic process, alkanesulphonate metabolism Subtypes: methanesulfonic acid metabolic process [GO:0018926], taurine metabolic process [GO:0019530], alkanesulfonate biosynthetic process [GO:0046305], GO:0046306, 6-sulfoquinovose(1-) catabolic process to glycerone phosphate and 3-sulfolactaldehyde [GO:0061720], 6-sulfoquinovose(1-) catabolic process to 3-sulfopropanediol(1-) [GO:0061721]